{
  "gene_symbol": "COL5A1-AS1",
  "gene_name": "Putative uncharacterized protein encoded by COL5A1-AS1",
  "term_label": "Unknown molecular function",
  "gene": "UniProtKB:Q5SY13",
  "term_id": "UNKNOWN:0001"
}